regulation of focal adhesion assembly [GO:0051893] (biological process) Definition: Any process that modulates the frequency, rate or extent of focal adhesion formation, the establishment and maturation of focal adhesions. Sources: GOC:ai Also known as: regulation of adhesion plaque assembly Relationships: is_a regulation of cell-matrix adhesion [GO:0001952]; is a type of regulation of cell-substrate junction assembly [GO:0090109]; RO_0002211 focal adhesion assembly [GO:0048041] Subtypes: positive regulation of focal adhesion assembly [GO:0051894], negative regulation of focal adhesion assembly [GO:0051895]